{
  "gene": "UniProtKB:Q969I3",
  "term_label": "glutamine metabolic process",
  "term_id": "GO:0006541",
  "gene_symbol": "GLYATL1",
  "gene_name": "Glycine N-acyltransferase-like protein 1"
}